symbiont-mediated disruption of host neutrophil extracellular traps [GO:0141144] (biological process) Relationships: is a type of symbiont-mediated disruption of host cellular anatomical structure [GO:0052008] Also known as: symbiont-mediated perturbation of host neutrophil extracellular traps References: PMID:16488875, PMID:21231972, PMID:25605868 Definition: A process in which a symbiont damages or impairs host neutrophil extracellular traps. The host is defined as the larger of the organisms involved in a symbiotic interaction.